{
  "gene": "UniProtKB:P01374",
  "gene_name": "Lymphotoxin-alpha",
  "term_label": "positive regulation of extrinsic apoptotic signaling pathway",
  "term_id": "GO:2001238",
  "gene_symbol": "LTA"
}